isobutyraldoxime O-methyltransferase activity [GO:0030763] (molecular function) Also known as: S-adenosyl-L-methionine:2-methylpropanal-oxime O-methyltransferase activity, S-adenosylmethionine:aldoxime O-methyltransferase activity, aldoxime O-methyltransferase activity, aldoxime methyltransferase activity Sources: EC:2.1.1.91, RHEA:10996 Relationships: is_a S-adenosylmethionine-dependent methyltransferase activity [GO:0008757] Definition: Catalysis of the reaction: 2-methylpropanal oxime + S-adenosyl-L-methionine = 2-methylpropanal O-methyloxime + S-adenosyl-L-homocysteine + H+.